negative regulation of voltage-gated potassium channel activity [GO:1903817] (biological process) Subtypes: negative regulation of delayed rectifier potassium channel activity [GO:1902260], negative regulation of inward rectifier potassium channel activity [GO:1903609] Relationships: is a type of GO:1901017; negatively regulates GO:0005249 Definition: Any process that stops, prevents or reduces the frequency, rate or extent of voltage-gated potassium channel activity. References: PMID:19219384 Sources: GOC:TermGenie, GO_REF:0000059 Also known as: down regulation of voltage gated potassium channel activity, down regulation of voltage-dependent potassium channel activity, down regulation of voltage-gated potassium channel activity, down regulation of voltage-gated potassium ion channel activity, down regulation of voltage-sensitive potassium channel, down-regulation of voltage gated potassium channel activity, down-regulation of voltage-dependent potassium channel activity, down-regulation of voltage-gated potassium channel activity, down-regulation of voltage-gated potassium ion channel activity, down-regulation of voltage-sensitive potassium channel, downregulation of voltage gated potassium channel activity, downregulation of voltage-dependent potassium channel activity, downregulation of voltage-gated potassium channel activity, downregulation of voltage-gated potassium ion channel activity, downregulation of voltage-sensitive potassium channel, negative regulation of voltage gated potassium channel activity, negative regulation of voltage-dependent potassium channel activity, negative regulation of voltage-gated potassium ion channel activity, negative regulation of voltage-sensitive potassium channel, inhibition of voltage gated potassium channel activity, inhibition of voltage-dependent potassium channel activity, inhibition of voltage-gated potassium channel activity, inhibition of voltage-gated potassium ion channel activity, inhibition of voltage-sensitive potassium channel